{
  "gene_symbol": "ACO1",
  "term_id": "GO:0006101",
  "term_label": "citrate metabolic process",
  "gene_name": "Cytoplasmic aconitate hydratase",
  "gene": "UniProtKB:P21399"
}